{
  "term_id": "GO:0035615",
  "term_label": "clathrin adaptor activity",
  "gene_symbol": "AP3M1",
  "gene": "UniProtKB:Q9Y2T2",
  "gene_name": "AP-3 complex subunit mu-1"
}